capitate projection [GO:0097387] (CC) Definition: Simple or compound process of epithelial glial cells with a spherical head that inserts into photoreceptor axons. Capitate projections have only been observed in Brachycera (flies). References: PMID:3098431 Sources: GOC:mc Relationships: is_a glial cell projection [GO:0097386]